{
  "gene_symbol": "GNA13",
  "term_id": "GO:0007189",
  "term_label": "adenylate cyclase-activating G protein-coupled receptor signaling pathway",
  "gene": "UniProtKB:Q14344",
  "gene_name": "Guanine nucleotide-binding protein subunit alpha-13"
}